{
  "term_id": "GO:0005635",
  "gene": "UniProtKB:Q9NXH8",
  "gene_symbol": "TOR4A",
  "term_label": "nuclear envelope",
  "gene_name": "Torsin-4A"
}